xyloglucan catabolic process [GO:2000899] (biological process) Sources: GOC:mengo_curators Relationships: is a type of glucan catabolic process [GO:0009251]; is a type of xyloglucan metabolic process [GO:0010411]; is a type of hemicellulose catabolic process [GO:2000895] Regulation: regulated by regulation of xyloglucan catabolic process [GO:2000951]; negatively regulated by negative regulation of xyloglucan catabolic process [GO:2000952]; positively regulated by positive regulation of xyloglucan catabolic process [GO:2000953] Definition: The chemical reactions and pathways resulting in the breakdown of a xyloglucan. Also known as: xyloglucan catabolism